{
  "gene_symbol": "CWC22",
  "gene": "UniProtKB:Q9HCG8",
  "term_id": "GO:0071013",
  "gene_name": "Pre-mRNA-splicing factor CWC22 homolog",
  "term_label": "catalytic step 2 spliceosome"
}